{
  "gene_symbol": "KIFC1",
  "gene": "UniProtKB:Q9BW19",
  "gene_name": "Kinesin-like protein KIFC1",
  "term_label": "mitotic spindle assembly",
  "term_id": "GO:0090307"
}